{
  "gene_name": "Zinc finger CCHC domain-containing protein 13",
  "term_label": "positive regulation of cytoplasmic translation",
  "gene_symbol": "ZCCHC13",
  "term_id": "GO:2000767",
  "gene": "UniProtKB:Q8WW36"
}